regulation of hepatocyte growth factor production [GO:0032646] (biological process) Definition: Any process that modulates the frequency, rate, or extent of hepatocyte growth factor production. References: PMID:1838014 Sources: GOC:mah Also known as: regulation of HGF production, regulation of scatter factor production, regulation of hepatocyte growth factor biosynthetic process Relationships: is a type of regulation of cytokine production [GO:0001817]; is a type of regulation of protein metabolic process [GO:0051246]; regulates hepatocyte growth factor production [GO:0032605] Subtypes: negative regulation of hepatocyte growth factor production [GO:0032686], GO:0032726